ATG2-ATG18 complex [GO:0062079] (cellular component) Relationships: is a type of membrane protein complex [GO:0098796]; is part of phagophore assembly site membrane [GO:0034045] References: PMID:23230146 Sources: GOC:bhm Definition: A protein complex essential for autophagy during nutrient deprivation, a catabolic process that sequesters undesired cellular material into autophagosomes for delivery to lysosomes for degradation. Contributes to nutrition homeostasis and damage control in eukaryotic cells. Functions at a late step of autophagosome formation for efficient completion of sequestration, probably through facilitating recruitment of ATG8-phosphatidylethanolamine (PE) to the preautophagosomal structure (PAS) and/or its protection from deconjugation by ATG4. Composed of ATG2 and ATG18 in Saccharomyces cerevisiae.